{
  "term_id": "GO:0045202",
  "gene_symbol": "MAP1B",
  "term_label": "synapse",
  "gene": "UniProtKB:P46821",
  "gene_name": "Microtubule-associated protein 1B"
}